NADPH:sulfur oxidoreductase activity [GO:0043914] (molecular function) References: PMID:17449625 Sources: GOC:jl Relationships: is_a oxidoreductase activity, acting on a sulfur group of donors [GO:0016667] Definition: Catalysis of the reaction: NADPH + H+ + sulfur = hydrogen sulfide + NADP+. Also known as: CoA-dependent NAD(P)H sulfur oxidoreductase activity, NAD(P)H elemental sulfur oxidoreductase activity, NAD(P)H sulfur oxidoreductase activity, NAD(P)H sulphur oxidoreductase activity, NAD(P)H:sulfur oxidoreductase activity, NADPH:sulphur oxidoreductase activity, NSR, coenzyme A-dependent NAD(P)H sulfur oxidoreductase activity